mRNA regulatory element binding translation repressor activity [GO:0000900] (molecular function) Also known as: translation repressor activity, nucleic acid binding, translation repressor activity, mRNA regulatory element binding Relationships: is a type of GO:0030371; has part mRNA binding [GO:0003729] Definition: Antagonizes the ribosome-mediated translation of mRNA into a polypeptide via direct binding (through a selective and non-covalent interaction) to nucleic acid. References: PMID:29061112, PMID:7523370 Sources: GOC:clt, GOC:vw